{
  "term_id": "GO:0005834",
  "term_label": "heterotrimeric G-protein complex",
  "gene": "UniProtKB:A0A1W2PPG7",
  "gene_symbol": "GNG14",
  "gene_name": "Putative guanine nucleotide-binding protein G(I)_G(S)_G(O) subunit gamma-14"
}